limb basal epidermal cell fate specification [GO:0060892] (biological process) Relationships: is_a GO:0009957; is_a GO:0060573; is part of limb epidermis stratification [GO:0060888]; is part of limb basal epidermal cell differentiation [GO:0060889] Definition: The process in which a cell becomes capable of differentiating autonomously into an limb basal epidermal cell in an environment that is neutral with respect to the developmental pathway; upon specification, the cell fate can be reversed. Sources: GOC:dph, GOC:sdb_2009, GOC:tb